{
  "term_label": "calcium ion binding",
  "gene_name": "Calmodulin-3",
  "term_id": "GO:0005509",
  "gene_symbol": "CALM3",
  "gene": "UniProtKB:P0DP25"
}